{
  "gene_symbol": "CTSW",
  "term_id": "GO:0051603",
  "gene_name": "Cathepsin W",
  "term_label": "proteolysis involved in protein catabolic process",
  "gene": "UniProtKB:P56202"
}